{
  "gene_symbol": "LAS1L",
  "gene_name": "Ribosomal biogenesis protein LAS1L",
  "term_label": "maturation of LSU-rRNA",
  "gene": "UniProtKB:Q9Y4W2",
  "term_id": "GO:0000470"
}